{
  "gene": "UniProtKB:Q6UXE8",
  "term_label": "external side of plasma membrane",
  "term_id": "GO:0009897",
  "gene_name": "Butyrophilin-like protein 3",
  "gene_symbol": "BTNL3"
}